{
  "gene_symbol": "PITX2",
  "term_label": "DNA-binding transcription factor activity, RNA polymerase II-specific",
  "term_id": "GO:0000981",
  "gene": "UniProtKB:Q99697",
  "gene_name": "Pituitary homeobox 2"
}